{
  "term_id": "GO:0005789",
  "term_label": "endoplasmic reticulum membrane",
  "gene": "UniProtKB:Q9Y5U9",
  "gene_symbol": "IER3IP1",
  "gene_name": "Immediate early response 3-interacting protein 1"
}